{
  "gene": "UniProtKB:O15297",
  "gene_name": "Protein phosphatase 1D",
  "gene_symbol": "PPM1D",
  "term_label": "regulation of intracellular signal transduction",
  "term_id": "GO:1902531"
}